{
  "gene_symbol": "PHTF2",
  "gene": "UniProtKB:Q8N3S3",
  "gene_name": "Protein PHTF2",
  "term_id": "UNKNOWN:0002",
  "term_label": "Unknown biological process"
}